{
  "gene_symbol": "ZNF304",
  "term_label": "DNA-binding transcription factor activity, RNA polymerase II-specific",
  "gene": "UniProtKB:Q9HCX3",
  "term_id": "GO:0000981",
  "gene_name": "Zinc finger protein 304"
}